{
  "term_id": "GO:0006338",
  "gene": "UniProtKB:P55198",
  "term_label": "chromatin remodeling",
  "gene_symbol": "MLLT6",
  "gene_name": "Protein AF-17"
}